glucarate catabolic process [GO:0019394] (biological process) Definition: The chemical reactions and pathways resulting in the breakdown of glucarate, the anion of glucaric acid. Sources: ISBN:0198506732 Also known as: glucarate breakdown, glucarate catabolism, glucarate degradation Relationships: is a type of GO:0019579 Subtypes: D-glucarate catabolic process [GO:0042838]